NADP binding [GO:0050661] (MF) Relationships: is a type of adenyl nucleotide binding [GO:0030554] Sources: GOC:ai Definition: Binding to nicotinamide-adenine dinucleotide phosphate, a coenzyme involved in many redox and biosynthetic reactions; binding may be to either the oxidized form, NADP+, or the reduced form, NADPH. Also known as: nicotinamide adenine dinucleotide phosphate binding, NADP or NADPH binding, NADP+ or NADPH binding Subtypes: NADP+ binding [GO:0070401], NADPH binding [GO:0070402]